eosinophil differentiation [GO:0030222] (biological process) Also known as: eosinophil cell differentiation, eosinophil cell development, eosinophil development Definition: The process in which a relatively unspecialized myeloid precursor cell acquires the specializes features of an eosinophil. Regulation: regulated by regulation of eosinophil differentiation [GO:0045643]; negatively regulated by negative regulation of eosinophil differentiation [GO:0045644]; positively regulated by positive regulation of eosinophil differentiation [GO:0045645] Relationships: is_a granulocyte differentiation [GO:0030851]; is a type of GO:0048468 Sources: GOC:add, GOC:mah